{
  "gene_symbol": "CISD3",
  "gene": "UniProtKB:P0C7P0",
  "gene_name": "CDGSH iron-sulfur domain-containing protein 3, mitochondrial",
  "term_id": "GO:0051537",
  "term_label": "2 iron, 2 sulfur cluster binding"
}